{
  "gene": "UniProtKB:A8K0S8",
  "term_label": "RNA polymerase II cis-regulatory region sequence-specific DNA binding",
  "gene_symbol": "MEIS3P2",
  "gene_name": "Putative homeobox protein Meis3-like 2",
  "term_id": "GO:0000978"
}